tauropine dehydrogenase activity [GO:0050325] (molecular function) Relationships: is a type of oxidoreductase activity, acting on the CH-NH group of donors, NAD or NADP as acceptor [GO:0016646] Also known as: 2-N-(D-1-carboxyethyl)taurine:NAD+ oxidoreductase (taurine-forming), N2-(D-1-carboxyethyl)taurine:NAD+ oxidoreductase (taurine-forming) Sources: EC:1.5.1.23, RHEA:12580 Definition: Catalysis of the reaction: H2O + NAD+ + tauropine = H+ + NADH + pyruvate + taurine.